planar dichotomous subdivision of terminal units involved in lung branching morphogenesis [GO:0060489] (biological process) Definition: The process in which a lung bud bifurcates parallel to the plane of the previous bud. Relationships: is a type of dichotomous subdivision of terminal units involved in lung branching [GO:0060448] Sources: GOC:dph, GOC:mtg_lung